L-tryptophan metabolic process [GO:0006568] (biological process) Relationships: is a type of GO:0009072; is a type of GO:0042430; is a type of GO:0170033; is a type of GO:0170039 Sources: ISBN:0198547684 Definition: The chemical reactions and pathways involving tryptophan, the chiral amino acid 2-amino-3-(1H-indol-3-yl)propanoic acid. Regulation: regulated by regulation of L-tryptophan metabolic process [GO:0090357]; positively regulated by positive regulation of L-tryptophan metabolic process [GO:0090358] Subtypes: L-tryptophan biosynthetic process [GO:0000162], L-tryptophan catabolic process [GO:0006569], GO:0009848, 'de novo' NAD+ biosynthetic process from L-tryptophan [GO:0034354], psilocybin biosynthetic process [GO:0140380] Also known as: tryptophan metabolic process, tryptophan metabolism